{
  "gene_symbol": "GABARAP",
  "gene_name": "Gamma-aminobutyric acid receptor-associated protein",
  "term_id": "GO:0000423",
  "gene": "UniProtKB:O95166",
  "term_label": "mitophagy"
}